{
  "term_label": "Unknown cellular component",
  "gene_name": "Protein FAM221B",
  "gene": "UniProtKB:A6H8Z2",
  "gene_symbol": "FAM221B",
  "term_id": "UNKNOWN:0003"
}